{
  "term_id": "UNKNOWN:0001",
  "gene": "UniProtKB:Q5QGS0",
  "gene_name": "Neurite extension and migration factor",
  "term_label": "Unknown molecular function",
  "gene_symbol": "NEXMIF"
}